delta6-acyl-lipid desaturase activity [GO:0102865] (molecular function) References: PMID:10848999 Sources: GOC:pz, RHEA:46536 Definition: Catalysis of the reaction: a gamma-linolenoyl-[glycerolipid] + 2 ferrocytochrome b5 + O2 + 2 H+ = a (9Z,12Z)-octadeca-9,12-dien-6-ynoyl-[glycerolipid] + 2 ferricytochrome b5 + 2 H2O. Relationships: is a type of oxidoreductase activity, acting on paired donors, with oxidation of a pair of donors resulting in the reduction of molecular oxygen to two molecules of water [GO:0016717]